{
  "gene": "UniProtKB:Q6PJ21",
  "gene_symbol": "SPSB3",
  "term_label": "SCF ubiquitin ligase complex",
  "gene_name": "SPRY domain-containing SOCS box protein 3",
  "term_id": "GO:0019005"
}